regulation of anterior head development [GO:2000742] (biological process) Sources: GOC:obol Definition: Any process that modulates the frequency, rate or extent of anterior head development. Relationships: is a type of regulation of developmental process [GO:0050793]; regulates anterior head development [GO:0097065] Subtypes: negative regulation of anterior head development [GO:2000743], positive regulation of anterior head development [GO:2000744]